{
  "term_id": "GO:0034472",
  "term_label": "snRNA 3'-end processing",
  "gene_name": "Integrator complex subunit 14",
  "gene_symbol": "INTS14",
  "gene": "UniProtKB:Q96SY0"
}